{
  "gene_name": "Protein NipSnap homolog 3A",
  "gene": "UniProtKB:Q9UFN0",
  "term_label": "Unknown molecular function",
  "gene_symbol": "NIPSNAP3A",
  "term_id": "UNKNOWN:0001"
}